{
  "term_label": "phosphorus-oxygen lyase activity",
  "term_id": "GO:0016849",
  "gene_name": "ADP-ribosyl cyclase_cyclic ADP-ribose hydrolase 2",
  "gene_symbol": "BST1",
  "gene": "UniProtKB:Q10588"
}